{
  "gene": "UniProtKB:P98155",
  "gene_name": "Very low-density lipoprotein receptor",
  "term_label": "Unknown biological process",
  "term_id": "UNKNOWN:0002",
  "gene_symbol": "VLDLR"
}